autophagy of peroxisome [GO:0030242] (biological process) Also known as: peroxisome degradation, peroxisome disassembly, pexophagy Definition: The process in which peroxisomes are delivered to a type of vacuole and degraded in response to changing nutrient conditions. References: PMID:10547367, PMID:20083110 Sources: GOC:autophagy Relationships: is a type of autophagy [GO:0006914] Subtypes: pexophagy [GO:0000425], micropexophagy [GO:0000426]